Fc receptor mediated stimulatory signaling pathway [GO:0002431] (biological process) Subtypes: GO:0038096, positive regulation of mast cell activation by Fc-epsilon receptor signaling pathway [GO:0038097] Relationships: is a type of immune response-activating cell surface receptor signaling pathway [GO:0002429] Also known as: Fc receptor mediated stimulatory signalling pathway, Fc-receptor mediated stimulatory signaling pathway Sources: GOC:add, GO_REF:0000022, ISBN:0781735149 Definition: The series of molecular signals generated as a consequence of a the binding of the Fc portion of an immunoglobulin by an Fc receptor capable of activating or perpetuating an immune response. The Fc portion of an immunoglobulin is its C-terminal constant region. Regulation: regulated by regulation of Fc receptor mediated stimulatory signaling pathway [GO:0060368]; positively regulated by positive regulation of Fc receptor mediated stimulatory signaling pathway [GO:0060369]